{
  "gene_name": "Mitoguardin 2",
  "gene": "UniProtKB:Q7L4E1",
  "gene_symbol": "MIGA2",
  "term_label": "Unknown cellular component",
  "term_id": "UNKNOWN:0003"
}